3-beta-hydroxysteroid dehydrogenase (NAD+)/C4-decarboxylase activity [GO:0102175] (molecular function) Definition: Catalysis of the reaction: a 3-beta-hydroxysteroid-4-alpha-carboxylate + NAD+ = a 3-oxosteroid + CO2 + NADH. Relationships: is a type of 3-beta-hydroxysteroid dehydrogenase [NAD(P)+]/C4-decarboxylase activity [GO:0000252] Sources: RHEA:34775